{
  "term_id": "GO:0030334",
  "gene_symbol": "TMSB10",
  "term_label": "regulation of cell migration",
  "gene": "UniProtKB:P63313",
  "gene_name": "Thymosin beta-10"
}